{
  "gene_symbol": "H2BW1",
  "term_label": "chromatin organization",
  "term_id": "GO:0006325",
  "gene": "UniProtKB:Q7Z2G1",
  "gene_name": "Histone H2B type W-T"
}